{
  "gene_name": "Peptidyl-prolyl cis-trans isomerase FKBP11",
  "term_id": "GO:0005783",
  "term_label": "endoplasmic reticulum",
  "gene_symbol": "FKBP11",
  "gene": "UniProtKB:Q9NYL4"
}